UMP kinase activity [GO:0033862] (molecular function) Sources: EC:2.7.4.22 Also known as: ATP:UMP phosphotransferase activity, PyrH, SmbA, UMP-kinase activity, UMPK, uridine monophosphate kinase activity Definition: Catalysis of the reaction: ATP + UMP = ADP + UDP. Relationships: is a type of nucleoside monophosphate kinase activity [GO:0050145]